viral tail assembly [GO:0098003] (biological process) Also known as: virus tail assembly, bacteriophage tail assembly Sources: GOC:bm, VZ:3955 Relationships: is a type of viral process [GO:0016032]; is part of virion assembly [GO:0019068] Definition: The aggregation, arrangement and bonding together of a set of components to form a virus tail.